{
  "gene_name": "Protein FAM216B",
  "term_label": "Unknown biological process",
  "gene": "UniProtKB:Q8N7L0",
  "term_id": "UNKNOWN:0002",
  "gene_symbol": "FAM216B"
}